{
  "term_label": "Unknown biological process",
  "gene": "UniProtKB:Q9Y2H5",
  "term_id": "UNKNOWN:0002",
  "gene_name": "Pleckstrin homology domain-containing family A member 6",
  "gene_symbol": "PLEKHA6"
}